{
  "gene_name": "Putative elongation factor 1-alpha-like 3",
  "term_label": "GTPase activity",
  "term_id": "GO:0003924",
  "gene_symbol": "EEF1A1P5",
  "gene": "UniProtKB:Q5VTE0"
}